negative regulation of glucose catabolic process to lactate via pyruvate [GO:1904024] (biological process) References: PMID:20935145 Sources: GOC:TermGenie, GOC:dph, GO_REF:0000058 Definition: Any process that stops, prevents or reduces the frequency, rate or extent of glucose catabolic process to lactate via pyruvate. Also known as: down regulation of glucose catabolic process to lactate via pyruvate, down regulation of glucose fermentation to lactate via pyruvate, down regulation of homofermentation, down regulation of homofermentative lactate fermentation, down regulation of homofermentative pathway, down regulation of homolactate fermentation, down regulation of homolactic fermentation, down-regulation of glucose catabolic process to lactate via pyruvate, down-regulation of glucose fermentation to lactate via pyruvate, down-regulation of homofermentation, down-regulation of homofermentative lactate fermentation, down-regulation of homofermentative pathway, down-regulation of homolactate fermentation, down-regulation of homolactic fermentation, downregulation of glucose catabolic process to lactate via pyruvate, downregulation of glucose fermentation to lactate via pyruvate, downregulation of homofermentation, downregulation of homofermentative lactate fermentation, downregulation of homofermentative pathway, downregulation of homolactate fermentation, downregulation of homolactic fermentation, negative regulation of glucose fermentation to lactate via pyruvate, negative regulation of homofermentation, negative regulation of homofermentative lactate fermentation, negative regulation of homofermentative pathway, negative regulation of homolactate fermentation, negative regulation of homolactic fermentation, inhibition of glucose catabolic process to lactate via pyruvate, inhibition of glucose fermentation to lactate via pyruvate, inhibition of homofermentation, inhibition of homofermentative lactate fermentation, inhibition of homofermentative pathway, inhibition of homolactate fermentation, inhibition of homolactic fermentation Relationships: is a type of negative regulation of catabolic process [GO:0009895]; is a type of negative regulation of carbohydrate metabolic process [GO:0045912]; is a type of negative regulation of small molecule metabolic process [GO:0062014]; is a type of negative regulation of fermentation [GO:1901003]; is a type of GO:1904023; negatively regulates glucose catabolic process to lactate via pyruvate [GO:0019661]